{
  "gene_name": "Protocadherin gamma-A11",
  "term_label": "cell adhesion",
  "term_id": "GO:0007155",
  "gene_symbol": "PCDHGA11",
  "gene": "UniProtKB:Q9Y5H2"
}